{
  "gene_symbol": "SCYGR3",
  "gene_name": "Small cysteine and glycine repeat-containing protein 3",
  "term_label": "Unknown molecular function",
  "gene": "UniProtKB:A0A286YF60",
  "term_id": "UNKNOWN:0001"
}